{
  "term_label": "Unknown cellular component",
  "gene_symbol": "CCDC102A",
  "gene_name": "Coiled-coil domain-containing protein 102A",
  "gene": "UniProtKB:Q96A19",
  "term_id": "UNKNOWN:0003"
}